{
  "term_label": "calcium ion sensor activity",
  "gene_symbol": "SYT8",
  "gene": "UniProtKB:Q8NBV8",
  "term_id": "GO:0061891",
  "gene_name": "Synaptotagmin-8"
}